{
  "gene_name": "Zinc finger protein 112",
  "gene_symbol": "ZNF112",
  "term_id": "GO:0006357",
  "gene": "UniProtKB:Q9UJU3",
  "term_label": "regulation of transcription by RNA polymerase II"
}